{
  "gene_symbol": "GARIN1B",
  "term_id": "UNKNOWN:0003",
  "gene": "UniProtKB:Q96KD3",
  "gene_name": "Golgi-associated RAB2 interactor protein 1B",
  "term_label": "Unknown cellular component"
}